{
  "term_id": "GO:0005886",
  "gene": "UniProtKB:O60636",
  "gene_name": "Tetraspanin-2",
  "term_label": "plasma membrane",
  "gene_symbol": "TSPAN2"
}